{
  "term_label": "homophilic cell-cell adhesion",
  "gene": "UniProtKB:Q15223",
  "gene_symbol": "NECTIN1",
  "gene_name": "Nectin-1",
  "term_id": "GO:0007156"
}